{
  "gene_name": "Tyrosine-protein phosphatase non-receptor type 14",
  "term_id": "GO:0001946",
  "gene_symbol": "PTPN14",
  "term_label": "lymphangiogenesis",
  "gene": "UniProtKB:Q15678"
}